{
  "gene_name": "Inactive tyrosine-protein kinase transmembrane receptor ROR1",
  "gene": "UniProtKB:Q01973",
  "term_id": "GO:0005886",
  "gene_symbol": "ROR1",
  "term_label": "plasma membrane"
}